mesonephric podocyte differentiation [GO:0061256] (biological process) Relationships: is a type of mesonephric glomerular epithelial cell differentiation [GO:0061250]; is a type of podocyte differentiation [GO:0072112] Definition: The process in which a relatively unspecialized cell acquires specialized features of a mesonephric glomerular visceral epithelial cell. A mesonephric glomerular visceral epithelial cell is a specialized epithelial cell that contains 'feet' that interdigitate with the 'feet' of other glomerular epithelial cells in the mesonephros. Also known as: mesonephric glomerular visceral epithelial cell differentiation Sources: GOC:mtg_kidney_jan10